imaginal disc growth [GO:0007446] (biological process) Definition: The increase in mass of imaginal discs by cell proliferation prior to metamorphosis. Imaginal discs are epithelial infoldings in the larvae of holometabolous insects that develop into adult structures (legs, antennae, wings, etc.) during metamorphosis from larval to adult form. Relationships: is a type of developmental growth [GO:0048589]; is part of imaginal disc development [GO:0007444] References: PMID:10679387 Sources: GOC:bf, GOC:jid Regulation: regulated by regulation of imaginal disc growth [GO:0045570]; negatively regulated by negative regulation of imaginal disc growth [GO:0045571]; RO_0002213 by positive regulation of imaginal disc growth [GO:0045572]